USH2 complex [GO:1990696] (cellular component) Definition: A protein complex composed of four proteins, loss of which results in Usher Syndrome type 2 (USH2 syndrome), a leading genetic cause of combined hearing and vision loss. This complex is conserved in many species; in mice, it is composed of USH2A, GPR98 (aka ADGRV1), WHRN, and PDZD7. Relationships: is a type of protein-containing complex [GO:0032991] Also known as: USH2 quaternary protein complex References: PMID:25406310 Sources: GOC:krc